SCF-Das1 ubiquitin ligase complex [GO:0097662] (cellular component) Definition: An SCF ubiquitin ligase complex in which the F-box protein is Das1 in S. cerevisiae. References: PMID:14747994 Sources: GOC:jd, GOC:vw Relationships: is a type of SCF ubiquitin ligase complex [GO:0019005]